{
  "gene": "UniProtKB:O95479",
  "gene_name": "GDH_6PGL endoplasmic bifunctional protein",
  "term_label": "glucose metabolic process",
  "term_id": "GO:0006006",
  "gene_symbol": "H6PD"
}